aminoglycoside antibiotic catabolic process [GO:0030649] (biological process) Subtypes: gentamycin catabolic process [GO:1901129], kanamycin catabolic process [GO:1901132], vistamycin catabolic process [GO:1901151], paromomycin catabolic process [GO:1901154], neomycin catabolic process [GO:1901157], daunorubicin catabolic process [GO:1901770] Also known as: aminoglycoside antibiotic breakdown, aminoglycoside antibiotic catabolism, aminoglycoside antibiotic degradation Definition: The chemical reactions and pathways resulting in the breakdown of an aminoglycoside antibiotic, any member of a group of broad spectrum antibiotics, of similar toxicity and pharmacology, that contain an aminodeoxysugar, an amino- or guanidino-substituted inositol ring, and one or more residues of other sugars. The group includes streptomycin, neomycin, framycetin, kanamycin, paromomycin, and gentamicin. Relationships: is a type of glycoside catabolic process [GO:0016139]; is a type of antibiotic catabolic process [GO:0017001] Sources: GOC:mah, ISBN:0198506732